{
  "gene_name": "CD109 antigen",
  "gene_symbol": "CD109",
  "term_id": "UNKNOWN:0003",
  "gene": "UniProtKB:Q6YHK3",
  "term_label": "Unknown cellular component"
}